{
  "gene_symbol": "TBX15",
  "gene_name": "T-box transcription factor TBX15",
  "gene": "UniProtKB:Q96SF7",
  "term_id": "GO:0001708",
  "term_label": "cell fate specification"
}